lateral mesodermal cell differentiation [GO:0048371] (biological process) Also known as: lateral mesoderm cell differentiation, lateral plate mesoderm cell differentiation, lateral plate mesodermal cell differentiation Definition: The process in which a relatively unspecialized cell acquires the specialized features of a lateral mesoderm cell. Relationships: is a type of GO:0048333; is part of GO:0048370 Sources: GOC:jid